{
  "gene_name": "N-terminal EF-hand calcium-binding protein 3",
  "gene_symbol": "NECAB3",
  "gene": "UniProtKB:Q96P71",
  "term_id": "UNKNOWN:0001",
  "term_label": "Unknown molecular function"
}